{
  "gene_symbol": "HEPN1",
  "term_label": "Unknown molecular function",
  "term_id": "UNKNOWN:0001",
  "gene_name": "Putative cancer susceptibility gene HEPN1 protein",
  "gene": "UniProtKB:Q6WQI6"
}